{
  "gene": "UniProtKB:Q0VG06",
  "gene_name": "Fanconi anemia core complex-associated protein 100",
  "gene_symbol": "FAAP100",
  "term_id": "GO:0005654",
  "term_label": "nucleoplasm"
}